{
  "gene_name": "Kelch-like protein 29",
  "gene": "UniProtKB:Q96CT2",
  "term_label": "ubiquitin-like ligase-substrate adaptor activity",
  "gene_symbol": "KLHL29",
  "term_id": "GO:1990756"
}